{
  "gene_symbol": "SPDYE8",
  "gene_name": "Putative speedy protein E8",
  "term_id": "GO:0019901",
  "term_label": "protein kinase binding",
  "gene": "UniProtKB:P0DUD1"
}